{
  "term_id": "GO:0036064",
  "term_label": "ciliary basal body",
  "gene_name": "Afadin- and alpha-actinin-binding protein",
  "gene_symbol": "SSX2IP",
  "gene": "UniProtKB:Q9Y2D8"
}